{
  "term_id": "GO:0019432",
  "gene_symbol": "LPIN1",
  "gene": "UniProtKB:Q14693",
  "gene_name": "Phosphatidate phosphatase LPIN1",
  "term_label": "triglyceride biosynthetic process"
}